{
  "gene_symbol": "APOBR",
  "term_label": "very-low-density lipoprotein particle receptor activity",
  "gene": "UniProtKB:Q0VD83",
  "term_id": "GO:0030229",
  "gene_name": "Apolipoprotein B receptor"
}